flower calyx development [GO:0048464] (biological process) Relationships: is a type of floral whorl development [GO:0048438] Definition: The process whose specific outcome is the progression of the flower calyx over time, from its formation to the mature structure. Sources: GOC:go_curators